ribonucleoprotein complex localization [GO:0071166] (biological process) Also known as: RNP localization, cellular ribonucleoprotein complex localization, establishment and maintenance of ribonucleoprotein complex localization, ribonucleoprotein complex localisation Definition: Any process in which a ribonucleoprotein complex is transported to, or maintained in, a specific location within a cell. Regulation: regulated by GO:2000197; negatively regulated by negative regulation of ribonucleoprotein complex localization [GO:2000198]; RO_0002213 by positive regulation of ribonucleoprotein complex localization [GO:2000199] Relationships: is a type of cellular localization [GO:0051641] Sources: GOC:mah